{
  "term_id": "GO:0005856",
  "gene_symbol": "CDC42EP3",
  "gene": "UniProtKB:Q9UKI2",
  "gene_name": "Cdc42 effector protein 3",
  "term_label": "cytoskeleton"
}